{
  "gene_name": "Cingulin-like protein 1",
  "gene": "UniProtKB:Q0VF96",
  "term_label": "Unknown molecular function",
  "term_id": "UNKNOWN:0001",
  "gene_symbol": "CGNL1"
}